regulation of death-inducing signaling complex assembly [GO:1903072] (biological process) Relationships: is a type of regulation of protein-containing complex assembly [GO:0043254]; regulates death-inducing signaling complex assembly [GO:0071550] Subtypes: negative regulation of death-inducing signaling complex assembly [GO:1903073] References: PMID:21785459 Sources: GOC:PARL, GOC:TermGenie, GOC:bf, GO_REF:0000058 Also known as: regulation of DD-mediated complex assembly, regulation of DISC assembly, regulation of DISC formation, regulation of death domain-mediated complex assembly, regulation of death domain-mediated complex assembly involved in extrinsic apoptotic pathway, regulation of death-inducing signaling complex formation, regulation of death-inducing signalling complex assembly Definition: Any process that modulates the frequency, rate or extent of death-inducing signaling complex assembly.